{
  "gene_name": "Alpha-S1-casein",
  "gene": "UniProtKB:P47710",
  "gene_symbol": "CSN1S1",
  "term_id": "GO:1903496",
  "term_label": "response to 11-deoxycorticosterone"
}